{
  "gene_name": "Intercellular adhesion molecule 2",
  "term_label": "integrin binding",
  "gene": "UniProtKB:P13598",
  "term_id": "GO:0005178",
  "gene_symbol": "ICAM2"
}